{
  "gene_symbol": "LINC03041",
  "term_label": "Unknown molecular function",
  "gene_name": "Putative uncharacterized protein encoded by LINC03041",
  "gene": "UniProtKB:A6NGG3",
  "term_id": "UNKNOWN:0001"
}